{
  "term_label": "protein-cysteine S-palmitoyltransferase activity",
  "gene_name": "Palmitoyltransferase ZDHHC2",
  "gene_symbol": "ZDHHC2",
  "term_id": "GO:0019706",
  "gene": "UniProtKB:Q9UIJ5"
}